{
  "gene_name": "STE20_SPS1-related proline-alanine-rich protein kinase",
  "gene": "UniProtKB:Q9UEW8",
  "term_id": "GO:0071474",
  "term_label": "cellular hyperosmotic response",
  "gene_symbol": "STK39"
}